{
  "gene_name": "Pleckstrin homology domain-containing family N member 1",
  "gene_symbol": "PLEKHN1",
  "gene": "UniProtKB:Q494U1",
  "term_label": "response to hypoxia",
  "term_id": "GO:0001666"
}